T cell meandering migration [GO:0120117] (biological process) Also known as: T cell meandering search, lymph node surveillance Definition: The random-like motility observed for T cells in lymph nodes which enhances surveillance of antigens presented by major histocompatibility complex (MHC) molecules on antigen presenting cells (APCs). References: PMID:25083865 Sources: GOC:add, GOC:krc Relationships: is a type of GO:0072678